{
  "gene": "UniProtKB:Q9NP74",
  "gene_name": "Palmdelphin",
  "term_id": "GO:0005737",
  "term_label": "cytoplasm",
  "gene_symbol": "PALMD"
}